{
  "gene_symbol": "MYLIP",
  "term_id": "GO:0006511",
  "gene": "UniProtKB:Q8WY64",
  "gene_name": "E3 ubiquitin-protein ligase MYLIP",
  "term_label": "ubiquitin-dependent protein catabolic process"
}